{
  "gene": "UniProtKB:Q6V0I7",
  "term_label": "adherens junction",
  "gene_symbol": "FAT4",
  "term_id": "GO:0005912",
  "gene_name": "Protocadherin Fat 4"
}